{
  "gene_symbol": "PRLHR",
  "term_id": "GO:0005886",
  "gene_name": "Prolactin-releasing peptide receptor",
  "gene": "UniProtKB:P49683",
  "term_label": "plasma membrane"
}